{
  "gene_name": "Zinc finger and BTB domain-containing protein 34",
  "term_id": "GO:0001817",
  "term_label": "regulation of cytokine production",
  "gene": "UniProtKB:Q8NCN2",
  "gene_symbol": "ZBTB34"
}